symbiont-mediated perturbation of host transcription [GO:0052026] (biological process) Definition: A process in which a symbiont alters or subverts transcription in its host. The host is defined as the larger of the organisms involved in a symbiotic interaction. Sources: GOC:mtg_pamgo_17jul06 Also known as: modulation by symbiont of host transcription Subtypes: GO:0039653, symbiont-mediated activation of host transcription [GO:1990216] Relationships: is a type of symbiont-mediated perturbation of host gene expression [GO:0039656]